{
  "gene_name": "B-cell lymphoma 6 protein",
  "gene_symbol": "BCL6",
  "term_label": "regulation of cell differentiation",
  "term_id": "GO:0045595",
  "gene": "UniProtKB:P41182"
}